negative regulation of dendritic spine maintenance [GO:1902951] (biological process) Definition: Any process that stops, prevents or reduces the frequency, rate or extent of dendritic spine maintenance. References: PMID:24328732 Sources: GOC:TermGenie, GOC:sjp, GO_REF:0000058 Relationships: is a type of negative regulation of cell projection organization [GO:0031345]; is a type of regulation of dendritic spine maintenance [GO:1902950]; negatively regulates dendritic spine maintenance [GO:0097062] Also known as: down regulation of dendritic spine maintenance, down-regulation of dendritic spine maintenance, downregulation of dendritic spine maintenance, inhibition of dendritic spine maintenance